{
  "gene_symbol": "ZNF66",
  "term_label": "Unknown cellular component",
  "term_id": "UNKNOWN:0003",
  "gene_name": "Putative zinc finger protein 66",
  "gene": "UniProtKB:Q6ZN08"
}